{
  "term_id": "UNKNOWN:0003",
  "gene_name": "T cell receptor alpha joining 30 (Fragment)",
  "gene_symbol": "TRAJ30",
  "gene": "UniProtKB:A0A075B6Y1",
  "term_label": "Unknown cellular component"
}